{
  "term_id": "GO:0005667",
  "gene_name": "Transcription factor 4",
  "gene_symbol": "TCF4",
  "term_label": "transcription regulator complex",
  "gene": "UniProtKB:P15884"
}